histone H1-4K34 acetyltransferase activity [GO:0140187] (molecular function) Relationships: is a type of histone H1 acetyltransferase activity [GO:0160262] Definition: Catalysis of the reaction: acetyl-CoA + histone H1-4 L-lysine (position 34) = CoA + histone H1-4 N6-acetyl-L-lysine (position 34). References: PMID:22465951